{
  "term_id": "GO:0050211",
  "gene_symbol": "COLGALT2",
  "gene_name": "Procollagen galactosyltransferase 2",
  "gene": "UniProtKB:Q8IYK4",
  "term_label": "procollagen galactosyltransferase activity"
}